{
  "gene_symbol": "IGF1R",
  "term_label": "axon",
  "gene_name": "Insulin-like growth factor 1 receptor",
  "gene": "UniProtKB:P08069",
  "term_id": "GO:0030424"
}